{
  "term_id": "GO:0031105",
  "gene": "UniProtKB:Q9P0V9",
  "gene_name": "Septin-10",
  "term_label": "septin complex",
  "gene_symbol": "SEPTIN10"
}